phosphatidylglycerol-phosphatidylethanolamine phosphatidyltransferase activity [GO:0090483] (molecular function) References: PMID:22988102 Definition: Catalysis of the reaction: phosphatidylglycerol + phosphatidylethanolamine = cardiolipin + ethanolamine. Also known as: cardiolipin synthase Relationships: is a type of phosphatidyltransferase activity [GO:0030572]